{
  "term_label": "regulation of apoptotic process",
  "gene": "UniProtKB:Q9UER7",
  "term_id": "GO:0042981",
  "gene_name": "Death domain-associated protein 6",
  "gene_symbol": "DAXX"
}